{
  "term_id": "GO:0005509",
  "gene_name": "Cytosolic phospholipase A2 epsilon",
  "gene": "UniProtKB:Q3MJ16",
  "term_label": "calcium ion binding",
  "gene_symbol": "PLA2G4E"
}